23S rRNA (adenine(1618)-N(6))-methyltransferase activity [GO:0052907] (molecular function) Relationships: is a type of rRNA (adenine-N6-)-methyltransferase activity [GO:0008988] Also known as: M(6)A(1618) activity, rRNA large subunit methyltransferase F activity Sources: RHEA:16497 Definition: Catalysis of the reaction: S-adenosyl-L-methionine + adenine(1618) in 23S rRNA = S-adenosyl-L-homocysteine + rRNA containing N(6)-methyladenine(1618) in 23S rRNA.